{
  "gene": "UniProtKB:A8MPX8",
  "gene_name": "Protein phosphatase 2C-like domain-containing protein 1",
  "term_label": "cytoplasm",
  "term_id": "GO:0005737",
  "gene_symbol": "PP2D1"
}